camera-type eye photoreceptor cell differentiation [GO:0060219] (biological process) Definition: The process in which a relatively unspecialized cell acquires the specialized features of a photoreceptor cell in a camera-type eye. Sources: GOC:ascb_2009, GOC:dph, GOC:tb Subtypes: retinal cone cell differentiation [GO:0042670], retinal rod cell differentiation [GO:0060221] Relationships: is a type of GO:0001754; is part of GO:0003407; is part of retina morphogenesis in camera-type eye [GO:0060042]